regulation of cell differentiation involved in tissue homeostasis [GO:0060786] (biological process) Sources: GOC:dph Definition: Any process that modulates the frequency, rate or extent of cell differentiation that contributes to the maintenance of a steady state of a cell type within a tissue. Relationships: is a type of regulation of cell differentiation [GO:0045595]; is part of homeostasis of number of cells within a tissue [GO:0048873]